{
  "term_id": "GO:2000147",
  "term_label": "positive regulation of cell motility",
  "gene_name": "14 kDa phosphohistidine phosphatase",
  "gene_symbol": "PHPT1",
  "gene": "UniProtKB:Q9NRX4"
}